{
  "gene_symbol": "VEGFB",
  "gene_name": "Vascular endothelial growth factor B",
  "term_id": "GO:0005615",
  "term_label": "extracellular space",
  "gene": "UniProtKB:P49765"
}